lateral line nerve glial cell morphogenesis involved in differentiation [GO:0048938] (biological process) Sources: GOC:dgh Definition: The process in which the structure of a glial cell in a lateral line nerve is generated and organized. This process occurs while the initially relatively unspecialized cell is acquiring the specialized features of a glial cell in a lateral line nerve. Subtypes: anterior lateral line nerve glial cell morphogenesis involved in differentiation [GO:0048940], GO:0048942 Relationships: is a type of cell morphogenesis [GO:0000902]; is part of lateral line nerve glial cell development [GO:0048937]